ATP:2-methylpropanoate phosphotransferase activity [GO:0047758] (molecular function) Sources: EC:2.7.2.14, RHEA:24156 Also known as: ATP:branched-chain-fatty-acid 1-phosphotransferase activity, branched-chain fatty acid kinase activity, branched-chain-fatty-acid kinase activity, isobutyrate kinase activity, ATP:2-methylpropanoate 1-phosphotransferase activity, ATP:2-methylpropanoate kinase activity, ATP:isobutyrate 1-phosphotransferase activity Relationships: is a type of kinase activity [GO:0016301]; is a type of phosphotransferase activity, carboxyl group as acceptor [GO:0016774] Definition: Catalysis of the reaction: 2-methylpropanoate + ATP = 2-methylpropanoyl phosphate + ADP + H+.